{
  "term_label": "Unknown molecular function",
  "gene_name": "NUT family member 2A",
  "gene_symbol": "NUTM2A",
  "gene": "UniProtKB:Q8IVF1",
  "term_id": "UNKNOWN:0001"
}